{
  "gene_name": "Keratin, type I cytoskeletal 28",
  "gene_symbol": "KRT28",
  "term_id": "GO:0030280",
  "gene": "UniProtKB:Q7Z3Y7",
  "term_label": "structural constituent of skin epidermis"
}